1-alkylglycerophosphocholine O-acyltransferase activity [GO:0047191] (MF) Definition: Catalysis of the reaction: 1-alkyl-sn-glycero-3-phosphocholine + acyl-CoA = 1-alkyl-2-acyl-sn-glycero-3-phosphocholine + CoA. Also known as: acyl-CoA:1-alkyl-sn-glycero-3-phosphocholine O-acyltransferase activity Relationships: is a type of O-acyltransferase activity [GO:0008374] Sources: EC:2.3.1.63, MetaCyc:2.3.1.63-RXN